{
  "term_id": "GO:0008168",
  "term_label": "methyltransferase activity",
  "gene": "UniProtKB:Q7Z4G4",
  "gene_symbol": "TRMT11",
  "gene_name": "tRNA (guanine(10)-N2)-methyltransferase homolog"
}